{
  "gene_symbol": "HLA-C",
  "gene_name": "HLA class I histocompatibility antigen, C alpha chain",
  "term_id": "GO:0030881",
  "gene": "UniProtKB:P10321",
  "term_label": "beta-2-microglobulin binding"
}